{
  "gene": "UniProtKB:Q6UWP2",
  "term_label": "Unknown molecular function",
  "gene_symbol": "DHRS11",
  "term_id": "UNKNOWN:0001",
  "gene_name": "Dehydrogenase_reductase SDR family member 11"
}